{
  "term_label": "Unknown molecular function",
  "gene_name": "Peroxisomal membrane protein 11A",
  "term_id": "UNKNOWN:0001",
  "gene": "UniProtKB:O75192",
  "gene_symbol": "PEX11A"
}